{
  "gene_symbol": "RHOA",
  "term_label": "GTP binding",
  "gene": "UniProtKB:P61586",
  "term_id": "GO:0005525",
  "gene_name": "Transforming protein RhoA"
}